{
  "gene_name": "72 kDa type IV collagenase",
  "term_label": "extracellular matrix organization",
  "gene_symbol": "MMP2",
  "gene": "UniProtKB:P08253",
  "term_id": "GO:0030198"
}